regulation of transmembrane transport [GO:0034762] (biological process) Also known as: regulation of membrane transport Subtypes: regulation of long-chain fatty acid import across plasma membrane [GO:0010746], regulation of D-glucose transmembrane transport [GO:0010827], GO:0022898, GO:0034763, positive regulation of transmembrane transport [GO:0034764], regulation of monoatomic ion transmembrane transport [GO:0034765], regulation of gluconate transmembrane transport [GO:0035430], GO:0090371, regulation of post-translational protein targeting to membrane, translocation [GO:0120235], regulation of sulfite transmembrane transport [GO:1900071], GO:1902267, regulation of (R)-carnitine transmembrane transport [GO:1902272], GO:1903789, regulation of protein import into chloroplast stroma [GO:1904215], GO:1905529, regulation of xenobiotic detoxification by transmembrane export across the plasma membrane [GO:1905699], regulation of phosphate transmembrane transport [GO:2000185], GO:2001148 Sources: GOC:mah Relationships: is a type of regulation of cellular process [GO:0050794]; is a type of regulation of transport [GO:0051049]; regulates transmembrane transport [GO:0055085] Definition: Any process that modulates the frequency, rate or extent of the directed movement of a solute from one side of a membrane to the other.